{
  "gene_name": "Forkhead box protein F1",
  "gene": "UniProtKB:Q12946",
  "term_id": "GO:0005634",
  "term_label": "nucleus",
  "gene_symbol": "FOXF1"
}